{
  "gene_name": "Olfactory receptor 5M8",
  "term_label": "olfactory receptor activity",
  "term_id": "GO:0004984",
  "gene": "UniProtKB:Q8NGP6",
  "gene_symbol": "OR5M8"
}